mammary gland duct regression in males [GO:0060641] (biological process) Definition: The process in which the epithelium of the mammary duct is destroyed in males. References: PMID:12558599 Sources: GOC:dph Relationships: is a type of anatomical structure regression [GO:0060033]; is part of mammary gland duct morphogenesis [GO:0060603]